negative regulation of sterigmatocystin biosynthetic process [GO:1900760] (BP) Also known as: down regulation of sterigmatocystin anabolism, down regulation of sterigmatocystin biosynthesis, down regulation of sterigmatocystin biosynthetic process, down regulation of sterigmatocystin formation, down regulation of sterigmatocystin synthesis, down-regulation of sterigmatocystin anabolism, down-regulation of sterigmatocystin biosynthesis, down-regulation of sterigmatocystin biosynthetic process, down-regulation of sterigmatocystin formation, down-regulation of sterigmatocystin synthesis, downregulation of sterigmatocystin anabolism, downregulation of sterigmatocystin biosynthesis, downregulation of sterigmatocystin biosynthetic process, downregulation of sterigmatocystin formation, downregulation of sterigmatocystin synthesis, inhibition of sterigmatocystin anabolism, inhibition of sterigmatocystin biosynthesis, inhibition of sterigmatocystin formation, inhibition of sterigmatocystin synthesis, negative regulation of sterigmatocystin anabolism, negative regulation of sterigmatocystin biosynthesis, negative regulation of sterigmatocystin formation, negative regulation of sterigmatocystin synthesis, inhibition of sterigmatocystin biosynthetic process Definition: Any process that stops, prevents or reduces the frequency, rate or extent of sterigmatocystin biosynthetic process. Sources: GOC:TermGenie, GOC:di Relationships: is a type of regulation of sterigmatocystin biosynthetic process [GO:0010913]; is a type of GO:1900377; negatively regulates sterigmatocystin biosynthetic process [GO:0045461]